{
  "gene_symbol": "SAGE1",
  "term_label": "snRNA 3'-end processing",
  "gene_name": "Sarcoma antigen 1",
  "gene": "UniProtKB:Q9NXZ1",
  "term_id": "GO:0034472"
}